{
  "term_id": "GO:0004796",
  "gene": "UniProtKB:P24557",
  "gene_name": "Thromboxane-A synthase",
  "gene_symbol": "TBXAS1",
  "term_label": "thromboxane-A synthase activity"
}